{
  "gene_symbol": "IL17RB",
  "gene": "UniProtKB:Q9NRM6",
  "term_id": "GO:0030368",
  "term_label": "interleukin-17 receptor activity",
  "gene_name": "Interleukin-17 receptor B"
}